{
  "gene_symbol": "BPIFA1",
  "term_id": "GO:0019731",
  "term_label": "antibacterial humoral response",
  "gene_name": "BPI fold-containing family A member 1",
  "gene": "UniProtKB:Q9NP55"
}